mercury ion transport [GO:0015694] (biological process) Also known as: mercury transport, mercuric ion transport Definition: The directed movement of mercury (Hg) ions into, out of or within a cell, or between cells, by means of some agent such as a transporter or pore. Sources: GOC:ai Relationships: is a type of transition metal ion transport [GO:0000041]; is a type of monoatomic cation transmembrane transport [GO:0098655]; is part of detoxification of mercury ion [GO:0050787]